{
  "gene": "UniProtKB:P01127",
  "term_label": "positive regulation of cell population proliferation",
  "term_id": "GO:0008284",
  "gene_name": "Platelet-derived growth factor subunit B",
  "gene_symbol": "PDGFB"
}